extraocular skeletal muscle development [GO:0002074] (biological process) Regulation: RO_0002211 by GO:0014725; negatively regulated by negative regulation of extraocular skeletal muscle development [GO:0014726]; positively regulated by positive regulation of extraocular skeletal muscle development [GO:0014727] Definition: The process whose specific outcome is the progression of the extraocular skeletal muscle over time, from its formation to the mature structure. The extraocular muscle is derived from cranial mesoderm and controls eye movements. The muscle begins its development with the differentiation of the muscle cells and ends with the mature muscle. An example of this process is found in Mus musculus. Relationships: is a type of skeletal muscle tissue development [GO:0007519]; is a type of skeletal muscle organ development [GO:0060538]; is part of GO:0043010 References: PMID:16638982 Sources: GOC:dph, GOC:mtg_muscle, GOC:mtg_sensu, MA:0001271